regulation of neurotransmitter receptor transport, endosome to postsynaptic membrane [GO:0099152] (biological process) References: PMID:20098723 Sources: GOC:dos Relationships: is a type of regulation of biological quality [GO:0065008]; is a type of GO:1902473; is a type of regulation of receptor localization to synapse [GO:1902683]; is a type of regulation of endosome to plasma membrane protein transport [GO:1905749]; regulates neurotransmitter receptor transport, endosome to postsynaptic membrane [GO:0098887] Definition: Any process that modulates the frequency, rate or extent of the directed movement of neurotransmitter receptor from the postsynaptic endosome to the postsynaptic membrane in transport vesicles.